{
  "gene_name": "Tudor domain-containing protein 15",
  "term_label": "Unknown biological process",
  "gene": "UniProtKB:B5MCY1",
  "term_id": "UNKNOWN:0002",
  "gene_symbol": "TDRD15"
}